{
  "gene": "UniProtKB:Q06278",
  "gene_name": "Aldehyde oxidase",
  "term_id": "GO:0004031",
  "term_label": "aldehyde oxidase activity",
  "gene_symbol": "AOX1"
}